{
  "gene_name": "Anillin",
  "term_label": "Unknown molecular function",
  "gene": "UniProtKB:Q9NQW6",
  "gene_symbol": "ANLN",
  "term_id": "UNKNOWN:0001"
}